{
  "gene_name": "Putative protein encoded by LINC02912",
  "term_label": "Unknown cellular component",
  "term_id": "UNKNOWN:0003",
  "gene": "UniProtKB:Q8N9X5",
  "gene_symbol": "LINC02912"
}